{
  "term_id": "GO:0005523",
  "term_label": "tropomyosin binding",
  "gene_name": "Tropomodulin-1",
  "gene_symbol": "TMOD1",
  "gene": "UniProtKB:P28289"
}